haltere morphogenesis [GO:0048735] (biological process) Sources: GOC:jid, GOC:rc Definition: The process in which the anatomical structures of a haltere are generated and organized. Relationships: is a type of imaginal disc-derived appendage morphogenesis [GO:0035114]; is_a GO:0035120; is part of haltere disc morphogenesis [GO:0007481]; is part of haltere development [GO:0007482]